symbiont-mediated suppression of host receptor-mediated signal transduction [GO:0075111] (BP) Definition: A process in which a virus interferes with, inhibits or disrupts a receptor-mediated signal transduction pathway in its host organism. The host is defined as the larger of the organisms involved in a symbiotic interaction. Sources: GOC:pamgo_curators Also known as: disruption of host receptor-mediated signal transduction, negative regulation by symbiont of host receptor-mediated signal transduction, suppression by symbiont of host receptor-mediated signal transduction Note: Note that this term is used to annotate gene products of the symbiont. To annotate host gene products, consider the biological process term "negative regulation by host of symbiont receptor-mediated signal transduction ; GO:0075080". Relationships: is a type of symbiont-mediated perturbation of host receptor-mediated signal transduction [GO:0075109]